{
  "gene_symbol": "PNRC2",
  "term_id": "GO:0000932",
  "gene_name": "Proline-rich nuclear receptor coactivator 2",
  "gene": "UniProtKB:Q9NPJ4",
  "term_label": "P-body"
}